{
  "gene_name": "CD164 sialomucin-like 2 protein",
  "term_id": "UNKNOWN:0001",
  "gene_symbol": "CD164L2",
  "gene": "UniProtKB:Q6UWJ8",
  "term_label": "Unknown molecular function"
}